ripoptosome [GO:0097342] (cellular component) Definition: A protein complex whose core components are the receptor-interacting serine/threonine-protein kinases RIPK1 and RIPK3 (also called RIP1 and RIP3). Formation of the ripoptosome can induce an extrinsic apoptotic signaling pathway or a necroptotic signaling pathway. The composition of this protein complex may depend on several factors including nature of the signal, cell type and more. References: PMID:22265414, PMID:22274400 Sources: GOC:bhm, GOC:mtg_apoptosis Also known as: TNFR1 complex II, Tnfr1-CII, necrosome Note: It has been shown that receptor-mediated necroptotic signaling pathway requires assembly of a ripoptosome protein complex consisting of caspase-8, caspase-10, Fas-associated death domain protein (FADD), casp8 and FADD-like apoptosis regulator (CFLAR) as well as the two receptor-interacting serine/threonine-protein kinases RIPK1 and RIPK3 (PMID:21737330). Optionally, depending on the receptor activated, this complex may contain TLR3 adaptor protein TRIF (PMID:21737330). Relationships: is a type of catalytic complex [GO:1902494]; is part of cytosol [GO:0005829]